dUTP biosynthetic process [GO:0006229] (biological process) Sources: ISBN:0198506732 Relationships: is a type of GO:0009212; is a type of pyrimidine deoxyribonucleotide biosynthetic process [GO:0009221]; is a type of dUTP metabolic process [GO:0046080] Definition: The chemical reactions and pathways resulting in the formation of dUTP, deoxyuridine (5'-)triphosphate. Also known as: dUTP anabolism, dUTP biosynthesis, dUTP formation, dUTP synthesis